{
  "term_id": "GO:0005789",
  "gene_name": "Elongation of very long chain fatty acids protein 6",
  "term_label": "endoplasmic reticulum membrane",
  "gene": "UniProtKB:Q9H5J4",
  "gene_symbol": "ELOVL6"
}